{
  "gene_name": "Transcription factor 4",
  "term_id": "GO:0000981",
  "gene": "UniProtKB:P15884",
  "gene_symbol": "TCF4",
  "term_label": "DNA-binding transcription factor activity, RNA polymerase II-specific"
}